{
  "gene_name": "Phosphoinositide 3-kinase regulatory subunit 6",
  "term_label": "1-phosphatidylinositol-3-kinase regulator activity",
  "term_id": "GO:0046935",
  "gene_symbol": "PIK3R6",
  "gene": "UniProtKB:Q5UE93"
}